afferent axon development in posterior lateral line nerve [GO:0048933] (biological process) References: PMID:15018940 Relationships: is a type of afferent axon development in lateral line nerve [GO:0048893]; is part of posterior lateral line nerve development [GO:0048918] Definition: The process whose specific outcome is the progression of an afferent axon in the posterior lateral line nerve over time from its formation to the mature structure. This process includes axonogenesis and pathfinding of the afferent axons in the posterior lateral line nerve.